response to 2-O-acetyl-1-O-hexadecyl-sn-glycero-3-phosphocholine [GO:1904316] (biological process) References: PMID:9321918 Sources: GOC:TermGenie, GO_REF:0000071 Also known as: response to PAF, response to platelet-activating factor Definition: Any process that results in a change in state or activity of a cell or an organism (in terms of movement, secretion, enzyme production, gene expression, etc.) as a result of a 2-O-acetyl-1-O-hexadecyl-sn-glycero-3-phosphocholine stimulus. Subtypes: GO:1904317 Relationships: is a type of response to lipid [GO:0033993]; is a type of GO:0045472; is a type of response to organophosphorus [GO:0046683]; is a type of response to nitrogen compound [GO:1901698]